autophagy [GO:0006914] (biological process) Subtypes: GO:0000422, macroautophagy [GO:0016236], microautophagy [GO:0016237], autophagy of peroxisome [GO:0030242], chaperone-mediated autophagy [GO:0061684], GO:0160155 Regulation: regulated by regulation of autophagy [GO:0010506]; negatively regulated by negative regulation of autophagy [GO:0010507]; positively regulated by positive regulation of autophagy [GO:0010508] Definition: The cellular catabolic process in which cells digest cellular materials, such as organelles and other macromolecular constituents, or non-self materials such as intracellular pathogens. Autophagy serves to provide essential nutrients under conditions of cellular stress; or can remodel intracellular structures during cell differentiation. Relationships: is a type of GO:0009056; is a type of process utilizing autophagic mechanism [GO:0061919]; BFO_0000051 transmembrane transport [GO:0055085] References: PMID:11099404, PMID:29455577, PMID:9412464 Sources: GOC:autophagy, ISBN:0198547684